{
  "gene_symbol": "JMY",
  "gene_name": "Junction-mediating and -regulatory protein",
  "gene": "UniProtKB:Q8N9B5",
  "term_label": "cytoplasm",
  "term_id": "GO:0005737"
}